{
  "term_id": "UNKNOWN:0001",
  "gene_symbol": "LENG8",
  "gene_name": "Leukocyte receptor cluster member 8",
  "term_label": "Unknown molecular function",
  "gene": "UniProtKB:Q96PV6"
}